regulation of heterochromatin organization [GO:0120261] (biological process) Definition: Any process that modulates the frequency, rate, extent or location of heterochromatin organization. Sources: GOC:krc Relationships: is a type of regulation of chromatin organization [GO:1902275]; regulates heterochromatin organization [GO:0070828] Subtypes: negative regulation of heterochromatin organization [GO:0120262], GO:0120263